{
  "gene_symbol": "TEX28",
  "gene_name": "Testis-specific protein TEX28",
  "term_label": "Unknown biological process",
  "gene": "UniProtKB:O15482",
  "term_id": "UNKNOWN:0002"
}